{
  "term_id": "GO:0004984",
  "gene_name": "Olfactory receptor 1E2",
  "term_label": "olfactory receptor activity",
  "gene": "UniProtKB:P47887",
  "gene_symbol": "OR1E2"
}